{
  "term_label": "Unknown biological process",
  "gene_symbol": "TMEM267",
  "gene": "UniProtKB:Q0VDI3",
  "term_id": "UNKNOWN:0002",
  "gene_name": "Transmembrane protein 267"
}